calcium-dependent protein serine/threonine phosphatase regulator activity [GO:0008597] (molecular function) Also known as: calcium-dependent protein serine/threonine phosphatase, intrinsic regulator activity Sources: GOC:ai Relationships: is a type of protein phosphatase regulator activity [GO:0019888]; regulates calcium-dependent protein serine/threonine phosphatase activity [GO:0004723] Definition: Binds to and modulates of the activity of the enzyme calcium-dependent protein serine/threonine phosphatase.